{
  "term_label": "glomerular filtration",
  "term_id": "GO:0003094",
  "gene_name": "TBC1 domain family member 8B",
  "gene": "UniProtKB:Q0IIM8",
  "gene_symbol": "TBC1D8B"
}